{
  "term_id": "GO:0004129",
  "gene_name": "Cytochrome c oxidase subunit 3",
  "gene": "UniProtKB:P00414",
  "term_label": "cytochrome-c oxidase activity",
  "gene_symbol": "MT-CO3"
}